{
  "term_id": "UNKNOWN:0003",
  "term_label": "Unknown cellular component",
  "gene": "UniProtKB:Q9BYQ0",
  "gene_name": "Keratin-associated protein 9-8",
  "gene_symbol": "KRTAP9-8"
}